transposable element silencing by heterochromatin formation [GO:0141005] (BP) References: PMID:25247314, PMID:28951459, PMID:32823517 Definition: A transposable element silencing mechanism involving heterochromatin assembly. Heterochromatin is a chromatin conformation that is refractory to transcription. Relationships: is a type of transposable element silencing [GO:0010526]; is a type of GO:0140719 Subtypes: transposable element silencing by piRNA-mediated heterochromatin formation [GO:0141006], transposable element silencing by siRNA-mediated heterochromatin formation [GO:0141007], transposable element silencing by siRNA-mediated DNA methylation [GO:0141010], GO:0141196 Also known as: retrotransposon silencing by heterochromatin formation